{
  "gene_name": "Nuclear valosin-containing protein-like",
  "term_label": "nucleus",
  "term_id": "GO:0005634",
  "gene_symbol": "NVL",
  "gene": "UniProtKB:O15381"
}